{
  "term_label": "double-strand break repair via break-induced replication",
  "gene_symbol": "MUS81",
  "term_id": "GO:0000727",
  "gene": "UniProtKB:Q96NY9",
  "gene_name": "Crossover junction endonuclease MUS81"
}